{
  "term_id": "GO:0106255",
  "term_label": "hydroperoxy icosatetraenoate isomerase activity",
  "gene_symbol": "ALOXE3",
  "gene_name": "Hydroperoxide isomerase ALOXE3",
  "gene": "UniProtKB:Q9BYJ1"
}